{
  "gene_name": "Myogenesis-regulating glycosidase",
  "term_label": "Unknown cellular component",
  "gene": "UniProtKB:Q6NSJ0",
  "term_id": "UNKNOWN:0003",
  "gene_symbol": "MYORG"
}